{
  "gene_name": "Dipeptidyl peptidase 1",
  "gene_symbol": "CTSC",
  "gene": "UniProtKB:P53634",
  "term_id": "GO:0051603",
  "term_label": "proteolysis involved in protein catabolic process"
}